{
  "term_id": "GO:0002062",
  "gene_symbol": "RUNX2",
  "term_label": "chondrocyte differentiation",
  "gene_name": "Runt-related transcription factor 2",
  "gene": "UniProtKB:Q13950"
}